{
  "gene_symbol": "PARVG",
  "gene": "UniProtKB:Q9HBI0",
  "term_label": "actin cytoskeleton organization",
  "term_id": "GO:0030036",
  "gene_name": "Gamma-parvin"
}